{
  "term_label": "extracellular space",
  "term_id": "GO:0005615",
  "gene_symbol": "CFHR5",
  "gene": "UniProtKB:Q9BXR6",
  "gene_name": "Complement factor H-related protein 5"
}